{
  "gene": "UniProtKB:Q8IUI4",
  "term_label": "Unknown cellular component",
  "gene_symbol": "SNX29P2",
  "gene_name": "Putative protein SNX29P2",
  "term_id": "UNKNOWN:0003"
}